chitin binding [GO:0008061] (molecular function) Relationships: is a type of carbohydrate derivative binding [GO:0097367] Definition: Binding to chitin, a linear polysaccharide consisting of beta-(1->4)-linked N-acetyl-D-glucosamine residues. Sources: GOC:jl, ISBN:0198506732